{
  "gene_name": "Rhotekin",
  "gene": "UniProtKB:Q9BST9",
  "term_id": "GO:0000281",
  "gene_symbol": "RTKN",
  "term_label": "mitotic cytokinesis"
}